{
  "term_label": "Unknown cellular component",
  "gene_name": "Motile sperm domain-containing protein 3",
  "gene_symbol": "MOSPD3",
  "gene": "UniProtKB:O75425",
  "term_id": "UNKNOWN:0003"
}